{
  "term_label": "Unknown cellular component",
  "gene_symbol": "SPDYE21",
  "gene_name": "Putative speedy protein E21",
  "term_id": "UNKNOWN:0003",
  "gene": "UniProtKB:A0A494C086"
}